{
  "term_id": "GO:0005886",
  "gene": "UniProtKB:O95858",
  "gene_symbol": "TSPAN15",
  "term_label": "plasma membrane",
  "gene_name": "Tetraspanin-15"
}